{
  "term_id": "GO:0005634",
  "gene": "UniProtKB:Q04727",
  "gene_symbol": "TLE4",
  "term_label": "nucleus",
  "gene_name": "Transducin-like enhancer protein 4"
}